{
  "gene_symbol": "GSTA1",
  "gene": "UniProtKB:P08263",
  "term_id": "GO:0006805",
  "gene_name": "Glutathione S-transferase A1",
  "term_label": "xenobiotic metabolic process"
}